histone H2AK119 ubiquitin ligase activity [GO:0140862] (molecular function) Also known as: histone H2A-K119 ubiquitin ligase activity, histone ubiquitin ligase activity (H2A-K119 specific) Note: Note that the residue position corresponds to the canonical human H2A2A histone (UniProtKB:Q6FI13); this residue is conserved across all eukaryotes. Residue 1 is the first residue following removal of the initiating Methionine (Met). Note that each histone is encoded by multiple genes, and sequences may vary across different genes within an organism. References: PMID:22844243, PMID:25470042, PMID:28624371 Relationships: is_a GO:0141053 Definition: Catalysis of the transfer of a ubiquitin molecule to histone 2A at the lysine-119 residue.